{
  "term_id": "GO:0016460",
  "gene_name": "Myosin-2",
  "gene": "UniProtKB:Q9UKX2",
  "gene_symbol": "MYH2",
  "term_label": "myosin II complex"
}